Golgi to lysosome transport [GO:0090160] (biological process) Definition: The directed movement of substances from the Golgi to lysosomes. Relationships: is a type of Golgi to vacuole transport [GO:0006896]; is a type of GO:0007041; is a type of cytosolic transport [GO:0016482] Sources: GOC:ascb_2009, GOC:dph, GOC:tb